{
  "gene_symbol": "FLVCR2",
  "gene": "UniProtKB:Q9UPI3",
  "gene_name": "Heme transporter FLVCR2",
  "term_label": "membrane",
  "term_id": "GO:0016020"
}